spindle pole body duplication [GO:0030474] (biological process) Sources: GOC:clt Also known as: spindle pole body assembly, spindle pole body biogenesis, spindle pole body biosynthesis, spindle pole body duplication associated with nuclear envelope, spindle pole body duplication in cytoplasm, spindle pole body formation, spindle pole body replication Relationships: is a type of cellular component assembly [GO:0022607]; is a type of spindle pole body organization [GO:0051300] Subtypes: mitotic spindle pole body duplication [GO:1903087] Definition: Construction of a new spindle pole body.